{
  "term_id": "GO:0006637",
  "gene_name": "Acyl-coenzyme A thioesterase 2, mitochondrial",
  "gene_symbol": "ACOT2",
  "term_label": "acyl-CoA metabolic process",
  "gene": "UniProtKB:P49753"
}